{
  "gene_name": "Keratin-associated protein 24-1",
  "gene_symbol": "KRTAP24-1",
  "term_id": "UNKNOWN:0003",
  "gene": "UniProtKB:Q3LI83",
  "term_label": "Unknown cellular component"
}